intracellular threonine homeostasis [GO:0090460] (biological process) Relationships: is a type of GO:0080144 Sources: GOC:tb Also known as: cellular threonine homeostasis, threonine homeostasis Definition: A homeostatic process involved in the maintenance of a steady state level of threonine within a cell.